{
  "gene": "UniProtKB:Q8IYS2",
  "gene_name": "Uncharacterized protein KIAA2013",
  "term_id": "UNKNOWN:0001",
  "term_label": "Unknown molecular function",
  "gene_symbol": "KIAA2013"
}